{
  "gene_name": "Probable ATP-dependent RNA helicase DDX6",
  "gene_symbol": "DDX6",
  "term_label": "P-body",
  "gene": "UniProtKB:P26196",
  "term_id": "GO:0000932"
}